{
  "gene_symbol": "SERPINH1",
  "term_label": "endoplasmic reticulum",
  "gene": "UniProtKB:P50454",
  "gene_name": "Serpin H1",
  "term_id": "GO:0005783"
}